cellular response to D-galactosamine [GO:1904422] (biological process) References: PMID:12057922 Sources: GOC:TermGenie, GO_REF:0000071 Definition: Any process that results in a change in state or activity of a cell (in terms of movement, secretion, enzyme production, gene expression, etc.) as a result of a D-galactosamine stimulus. Relationships: is a type of cellular response to oxygen-containing compound [GO:1901701]; is a type of response to D-galactosamine [GO:1904421]